{
  "term_id": "GO:0072659",
  "gene": "UniProtKB:Q96G30",
  "gene_symbol": "MRAP2",
  "term_label": "protein localization to plasma membrane",
  "gene_name": "Melanocortin-2 receptor accessory protein 2"
}